signaling receptor ligand precursor processing [GO:0140448] (biological process) Also known as: ligand maturation, signal maturation References: PMID:29247995 Definition: The cleavage of a peptide bond in a precursor form of a signaling receptor ligand, resulting in the mature (active) form of the ligand. Subtypes: peptide hormone processing [GO:0016486], neuropeptide processing [GO:0061837], cytokine precursor processing [GO:0140447] Relationships: is a type of GO:0016485